{
  "term_label": "lymphocyte differentiation",
  "gene": "UniProtKB:P31785",
  "gene_symbol": "IL2RG",
  "gene_name": "Cytokine receptor common subunit gamma",
  "term_id": "GO:0030098"
}